{
  "gene_name": "DAZ-associated protein 1",
  "gene": "UniProtKB:Q96EP5",
  "term_id": "GO:1990904",
  "gene_symbol": "DAZAP1",
  "term_label": "ribonucleoprotein complex"
}